{
  "gene_name": "Cytoplasmic dynein 1 light intermediate chain 1",
  "gene": "UniProtKB:Q9Y6G9",
  "gene_symbol": "DYNC1LI1",
  "term_id": "GO:0000226",
  "term_label": "microtubule cytoskeleton organization"
}